{
  "term_id": "UNKNOWN:0003",
  "gene_name": "Putative microRNA 17 host gene protein",
  "gene_symbol": "MIR17HG",
  "term_label": "Unknown cellular component",
  "gene": "UniProtKB:Q75NE6"
}